{
  "term_label": "cell morphogenesis",
  "gene_symbol": "CDH24",
  "gene_name": "Cadherin-24",
  "gene": "UniProtKB:Q86UP0",
  "term_id": "GO:0000902"
}